{
  "term_label": "sensory perception of sound",
  "gene": "UniProtKB:O94898",
  "term_id": "GO:0007605",
  "gene_name": "Leucine-rich repeats and immunoglobulin-like domains protein 2",
  "gene_symbol": "LRIG2"
}